{
  "gene_symbol": "PGLYRP2",
  "gene_name": "N-acetylmuramoyl-L-alanine amidase",
  "term_label": "N-acetylmuramoyl-L-alanine amidase activity",
  "gene": "UniProtKB:Q96PD5",
  "term_id": "GO:0008745"
}